{
  "term_label": "proton-transporting ATP synthase complex",
  "term_id": "GO:0045259",
  "gene_symbol": "ATP5MC3",
  "gene": "UniProtKB:P48201",
  "gene_name": "ATP synthase F(0) complex subunit C3, mitochondrial"
}